guanidinopropionase activity [GO:0047972] (molecular function) Definition: Catalysis of the reaction: 3-guanidinopropanoate + H2O = beta-alanine + urea. Relationships: is_a hydrolase activity, acting on carbon-nitrogen (but not peptide) bonds, in linear amidines [GO:0016813] Also known as: 3-guanidinopropanoate amidinopropionase activity, GPH, GPase activity Sources: EC:3.5.3.17, RHEA:16029